negative regulation of astrocyte differentiation [GO:0048712] (biological process) Definition: Any process that stops, prevents, or reduces the frequency, rate or extent of astrocyte differentiation. Subtypes: negative regulation of astrocyte activation [GO:0061889] Relationships: is a type of GO:0045686; is a type of regulation of astrocyte differentiation [GO:0048710]; negatively regulates astrocyte differentiation [GO:0048708] References: PMID:15139015 Sources: GOC:vp Also known as: down regulation of astrocyte differentiation, down-regulation of astrocyte differentiation, downregulation of astrocyte differentiation, inhibition of astrocyte differentiation